developmental induction [GO:0031128] (biological process) References: PMID:24503535 Sources: GOC:cjm, GOC:dph, GOC:mah Definition: A developmental process involving two tissues in which one tissue (the inducer) produces a signal that directs cell fate commitment of cells in the second tissue (the responder). Relationships: is a type of developmental process [GO:0032502]; BFO_0000051 cell-cell signaling involved in cell fate commitment [GO:0045168] Subtypes: organ induction [GO:0001759], forebrain induction by the anterior neural ridge [GO:0022000], GO:0031129, lens induction in camera-type eye [GO:0060235], GO:0072034